N-substituted formamide deformylase activity [GO:0033966] (molecular function) Sources: EC:3.5.1.91 Relationships: is a type of hydrolase activity, acting on carbon-nitrogen (but not peptide) bonds, in linear amides [GO:0016811] Definition: Catalysis of the reaction: N-benzylformamide + H2O = formate + benzylamine. Also known as: N-benzylformamide amidohydrolase activity, NfdA